{
  "term_label": "DNA-binding transcription factor activity, RNA polymerase II-specific",
  "gene_name": "Hairy_enhancer-of-split related with YRPW motif protein 2",
  "term_id": "GO:0000981",
  "gene": "UniProtKB:Q9UBP5",
  "gene_symbol": "HEY2"
}